{
  "gene": "UniProtKB:Q02742",
  "gene_name": "Beta-1,3-galactosyl-O-glycosyl-glycoprotein beta-1,6-N-acetylglucosaminyltransferase",
  "gene_symbol": "GCNT1",
  "term_id": "UNKNOWN:0003",
  "term_label": "Unknown cellular component"
}